negative regulation of rRNA processing [GO:2000233] (biological process) Definition: Any process that stops, prevents, or reduces the frequency, rate or extent of rRNA processing. Also known as: negative regulation of 35S primary transcript processing Relationships: is a type of GO:0010629; is a type of GO:0051253; is a type of negative regulation of ribosome biogenesis [GO:0090071]; is_a regulation of rRNA processing [GO:2000232]; RO_0002212 GO:0006364 Sources: GOC:mah